{
  "gene": "UniProtKB:Q9BY67",
  "gene_symbol": "CADM1",
  "gene_name": "Cell adhesion molecule 1",
  "term_id": "GO:0007156",
  "term_label": "homophilic cell-cell adhesion"
}